lateral root morphogenesis [GO:0010102] (biological process) Definition: The process in which the anatomical structures of a lateral root are generated and organized. A lateral root is one formed from pericycle cells located on the xylem radius of the root, as opposed to the initiation of the main root from the embryo proper. Relationships: is a type of post-embryonic root morphogenesis [GO:0010101]; is part of lateral root development [GO:0048527] Sources: GOC:tair_curators